{
  "gene_symbol": "IGKV3D-15",
  "term_id": "GO:0019814",
  "gene": "UniProtKB:A0A087WSY6",
  "term_label": "immunoglobulin complex",
  "gene_name": "Immunoglobulin kappa variable 3D-15"
}